collagenous component of interstitial matrix [GO:0140152] (CC) Relationships: is a type of GO:0030312; is part of solid phase of interstitial matrix [GO:0140151] References: PMID:12064927, PMID:17550969, PMID:21421911, PMID:28101870, PMID:39223427 Definition: Main components of the interstitial matrix solid phase, including fibrillar and fibril-associated collagens.